{
  "gene": "UniProtKB:P0CG08",
  "term_id": "GO:0008308",
  "gene_name": "Golgi pH regulator B",
  "term_label": "voltage-gated monoatomic anion channel activity",
  "gene_symbol": "GPR89B"
}